{
  "gene_symbol": "NLGN4X",
  "gene": "UniProtKB:Q8N0W4",
  "term_label": "Unknown biological process",
  "term_id": "UNKNOWN:0002",
  "gene_name": "Neuroligin-4, X-linked"
}